vibriobactin biosynthetic process [GO:0019537] (biological process) Also known as: vibriobactin anabolism, vibriobactin biosynthesis, vibriobactin formation, vibriobactin synthesis, vibriobactin biosynthetic process, peptide formation, vibriobactin biosynthetic process, peptide modification Relationships: is_a vibriobactin metabolic process [GO:0019536]; is a type of amide biosynthetic process [GO:0043604] Definition: The chemical reactions and pathways resulting in the formation of vibriobactin, the major siderophore produced by Vibrio cholerae. References: PMID:11112537 Sources: GOC:jl